{
  "gene_symbol": "MAN1C1",
  "term_id": "GO:0005783",
  "term_label": "endoplasmic reticulum",
  "gene_name": "Mannosyl-oligosaccharide 1,2-alpha-mannosidase IC",
  "gene": "UniProtKB:Q9NR34"
}